{
  "term_id": "GO:0006506",
  "gene": "UniProtKB:Q9BRR3",
  "gene_symbol": "PGAP4",
  "term_label": "GPI anchor biosynthetic process",
  "gene_name": "Post-GPI attachment to proteins factor 4"
}